negative regulation of capsule organization [GO:1901914] (biological process) Definition: Any process that stops, prevents or reduces the frequency, rate or extent of capsule organization. Relationships: is a type of GO:0051129; is a type of GO:1901913; negatively regulates capsule organization [GO:0045230] Also known as: down regulation of capsule organisation, down regulation of capsule organization, down-regulation of capsule organisation, down-regulation of capsule organization, downregulation of capsule organisation, downregulation of capsule organization, negative regulation of capsule organisation, inhibition of capsule organisation, inhibition of capsule organization, down regulation of capsule organization and biogenesis, down-regulation of capsule organization and biogenesis, downregulation of capsule organization and biogenesis, inhibition of capsule organization and biogenesis, negative regulation of capsule organization and biogenesis Sources: GOC:TermGenie, GOC:di